positive regulation of male gonad development [GO:2000020] (biological process) Sources: GOC:obol Relationships: is a type of positive regulation of gonad development [GO:1905941]; is a type of regulation of male gonad development [GO:2000018]; positively regulates male gonad development [GO:0008584] Also known as: positive regulation of testicular development, positive regulation of testis development Definition: Any process that activates or increases the frequency, rate or extent of male gonad development.